{
  "term_id": "GO:0070306",
  "gene_name": "Phospholipase A and acyltransferase 3",
  "gene_symbol": "PLAAT3",
  "term_label": "lens fiber cell differentiation",
  "gene": "UniProtKB:P53816"
}